{
  "gene_symbol": "BGLAP",
  "gene_name": "Osteocalcin",
  "term_label": "extracellular region",
  "term_id": "GO:0005576",
  "gene": "UniProtKB:P02818"
}